{
  "gene_name": "Kallikrein-10",
  "term_id": "GO:0051604",
  "gene_symbol": "KLK10",
  "term_label": "protein maturation",
  "gene": "UniProtKB:O43240"
}